{
  "gene_symbol": "JUP",
  "term_id": "GO:0098609",
  "gene": "UniProtKB:P14923",
  "term_label": "cell-cell adhesion",
  "gene_name": "Junction plakoglobin"
}